{
  "gene": "UniProtKB:Q9HAW8",
  "gene_symbol": "UGT1A10",
  "term_label": "enzyme inhibitor activity",
  "term_id": "GO:0004857",
  "gene_name": "UDP-glucuronosyltransferase 1A10"
}